{
  "gene": "UniProtKB:Q9BZW2",
  "term_id": "GO:0015382",
  "term_label": "sodium:sulfate symporter activity",
  "gene_symbol": "SLC13A1",
  "gene_name": "Solute carrier family 13 member 1"
}